{
  "term_id": "GO:0007155",
  "gene_symbol": "IZUMO1R",
  "gene": "UniProtKB:A6ND01",
  "term_label": "cell adhesion",
  "gene_name": "Sperm-egg fusion protein Juno"
}